detection of yeast [GO:0001879] (biological process) Definition: The series of events in which a stimulus from a yeast is received and converted into a molecular signal. Relationships: is a type of GO:0001878; is a type of detection of fungus [GO:0016046] References: PMID:14707091